{
  "term_label": "DNA-binding transcription factor activity, RNA polymerase II-specific",
  "gene_name": "Zinc finger protein 679",
  "gene_symbol": "ZNF679",
  "term_id": "GO:0000981",
  "gene": "UniProtKB:Q8IYX0"
}